{
  "gene_name": "Uncharacterized protein",
  "term_id": "UNKNOWN:0003",
  "term_label": "Unknown cellular component",
  "gene_symbol": "LOC122394732",
  "gene": "UniProtKB:A0A1B0GW15"
}